{
  "term_label": "Unknown molecular function",
  "gene": "UniProtKB:Q8IZL8",
  "gene_symbol": "PELP1",
  "term_id": "UNKNOWN:0001",
  "gene_name": "Proline-, glutamic acid- and leucine-rich protein 1"
}